effector-mediated perturbation of host process by symbiont [GO:0140418] (biological process) Also known as: effector mediated modulation of host process by symbiont, effector triggered modulation of host process by symbiont, effector-dependent modulation of host process by symbiont, effector-mediated modulation of host process by symbiont References: PMID:21467214 Subtypes: effector-mediated perturbation of host defenses by symbiont [GO:0140415], effector-mediated induction of cell cycle reactivation in host [GO:0141017] Definition: A process mediated by a molecule secreted by a symbiont that results in the modulation (either activation or suppression) of a host structure or process. The host is defined as the larger of the organisms involved in a symbiotic interaction. Relationships: is a type of symbiont-mediated perturbation of host process [GO:0044003]